{
  "gene_symbol": "IRF9",
  "term_id": "GO:0005634",
  "gene_name": "Interferon regulatory factor 9",
  "term_label": "nucleus",
  "gene": "UniProtKB:Q00978"
}